interleukin-21 binding [GO:0019977] (molecular function) Definition: Binding to interleukin-21. Relationships: is a type of GO:0019955 Also known as: IL-21 binding Sources: GOC:jl